D-glucarate biosynthetic process [GO:0042837] (biological process) Relationships: is a type of carbohydrate biosynthetic process [GO:0016051]; is a type of glucarate biosynthetic process [GO:0019393]; is a type of D-glucarate metabolic process [GO:0042836] Sources: GOC:jsg, GOC:mah, ISBN:0198506732 Definition: The chemical reactions and pathways resulting in the formation of D-glucarate, the D-enantiomer of glucarate. Also known as: D-glucarate anabolism, D-glucarate biosynthesis, D-glucarate formation, D-glucarate synthesis, saccharate biosynthesis, saccharate biosynthetic process